UDP-N-acetylglucosamine biosynthetic process [GO:0006048] (biological process) Sources: GOC:ai Definition: The chemical reactions and pathways resulting in the formation of UDP-N-acetylglucosamine, a substance composed of N-acetylglucosamine, a common structural unit of oligosaccharides, in glycosidic linkage with uridine diphosphate. Relationships: is a type of UDP-N-acetylglucosamine metabolic process [GO:0006047]; is a type of nucleotide-sugar biosynthetic process [GO:0009226]; is a type of GO:0046349 Also known as: UDP-GlcNAc biosynthesis, UDP-GlcNAc biosynthetic process, UDP-N-acetylglucosamine anabolism, UDP-N-acetylglucosamine biosynthesis, UDP-N-acetylglucosamine formation, UDP-N-acetylglucosamine synthesis Regulation: regulated by GO:0106278; negatively regulated by negative regulation of UDP-N-acetylglucosamine biosynthetic process [GO:0106279]; positively regulated by positive regulation of UDP-N-acetylglucosamine biosynthetic process [GO:0106280]